inhibitory killer cell immunoglobulin-like receptor signaling pathway [GO:0002771] (biological process) References: PMID:15771571 Sources: GOC:add, ISBN:0781735149 Definition: The series of molecular signals initiated by an extracellular ligand binding to a inhibitory killer cell immunoglobulin-like receptor capable of inhibiting an immune effector process contributing to an immune response. Relationships: is a type of GO:0002767 Also known as: KIR signaling pathway, inhibitory killer cell immunoglobulin-like receptor signalling pathway, killer cell inhibitory receptor signaling pathway